thiohydroximate beta-D-glucosyltransferase activity [GO:0047251] (molecular function) Also known as: N-hydroxythioamide S-beta-glucosyltransferase activity, UDP-glucose:N-hydroxy-2-phenylethanethioamide S-beta-D-glucosyltransferase activity, UDP-glucose:thiohydroximate S-beta-D-glucosyltransferase activity, UDPG:thiohydroximate glucosyltransferase activity, desulfoglucosinolate-uridine diphosphate glucosyltransferase activity, thiohydroximate S-glucosyltransferase activity, thiohydroximate glucosyltransferase activity, uridine diphosphoglucose-thiohydroximate glucosyltransferase activity Sources: EC:2.4.1.195 Relationships: is a type of UDP-glucosyltransferase activity [GO:0035251] Definition: Catalysis of the reaction: phenylthioacetohydroximate + UDP-D-glucose = desulfoglucotropeolin + UDP.